{
  "term_label": "actin cytoskeleton organization",
  "gene_name": "F-actin-capping protein subunit alpha-1",
  "gene_symbol": "CAPZA1",
  "gene": "UniProtKB:P52907",
  "term_id": "GO:0030036"
}